{
  "gene_symbol": "CLEC4F",
  "term_id": "GO:0006955",
  "gene_name": "C-type lectin domain family 4 member F",
  "term_label": "immune response",
  "gene": "UniProtKB:Q8N1N0"
}